spermatocyte division [GO:0048137] (biological process) Also known as: spermatocyte cell division Relationships: is a type of cell division [GO:0051301]; is part of spermatogenesis [GO:0007283] Sources: GOC:jid, GOC:pr, ISBN:0879694238 Definition: The meiotic divisions undergone by the primary and secondary spermatocytes to produce haploid spermatids.